{
  "gene_name": "Protein RUFY3",
  "gene": "UniProtKB:Q7L099",
  "term_label": "regulation of axonogenesis",
  "term_id": "GO:0050770",
  "gene_symbol": "RUFY3"
}